{
  "term_id": "GO:0061630",
  "gene_symbol": "RNF180",
  "gene": "UniProtKB:Q86T96",
  "gene_name": "E3 ubiquitin-protein ligase RNF180",
  "term_label": "ubiquitin protein ligase activity"
}